male courtship behavior, veined wing vibration [GO:0016545] (biological process) Relationships: is_a GO:0048065 References: PMID:11092827 Sources: GOC:mtg_sensu Definition: The process during courtship where the male insect vibrates his wings. An example of this is found in Drosophila melanogaster. Also known as: male courtship behaviour, veined wing vibration, male courtship behavior, wing vibration, male courtship behaviour, wing vibration